{
  "gene": "UniProtKB:O43790",
  "term_label": "keratin filament",
  "term_id": "GO:0045095",
  "gene_symbol": "KRT86",
  "gene_name": "Keratin, type II cuticular Hb6"
}